{
  "term_id": "GO:0005634",
  "gene": "UniProtKB:Q9UL17",
  "term_label": "nucleus",
  "gene_symbol": "TBX21",
  "gene_name": "T-box transcription factor TBX21"
}